response to quetiapine [GO:0097335] (biological process) Sources: GOC:pr Definition: Any process that results in a change in state or activity of a cell or an organism (in terms of movement, secretion, enzyme production, gene expression, etc.) as a result of a quetiapine stimulus. Relationships: is a type of response to nitrogen compound [GO:1901698]